{
  "gene_symbol": "AIDA",
  "term_id": "GO:0035091",
  "gene": "UniProtKB:Q96BJ3",
  "term_label": "phosphatidylinositol binding",
  "gene_name": "Axin interactor, dorsalization-associated protein"
}